positive regulation of microvillus length [GO:1903983] (biological process) Relationships: is a type of positive regulation of cell projection organization [GO:0031346]; is a type of regulation of microvillus length [GO:0032532] References: PMID:22114352 Sources: GOC:als Also known as: up regulation of regulation of microvillus length, up-regulation of regulation of microvillus length, upregulation of regulation of microvillus length, activation of regulation of microvillus length Definition: A process that increases the length of a microvillus.